{
  "term_label": "N-acetylglucosamine-6-sulfatase activity",
  "gene": "UniProtKB:Q8IWU6",
  "gene_name": "Extracellular sulfatase Sulf-1",
  "gene_symbol": "SULF1",
  "term_id": "GO:0008449"
}